{
  "gene_symbol": "TAS2R10",
  "gene": "UniProtKB:Q9NYW0",
  "gene_name": "Taste receptor type 2 member 10",
  "term_id": "UNKNOWN:0002",
  "term_label": "Unknown biological process"
}